{
  "gene": "UniProtKB:Q9BZE3",
  "term_label": "DNA-binding transcription factor activity, RNA polymerase II-specific",
  "gene_name": "BarH-like 1 homeobox protein",
  "gene_symbol": "BARHL1",
  "term_id": "GO:0000981"
}